{
  "gene_symbol": "DFFB",
  "term_label": "DNA nuclease activity",
  "gene_name": "DNA fragmentation factor subunit beta",
  "term_id": "GO:0004536",
  "gene": "UniProtKB:O76075"
}